{
  "term_id": "GO:0005737",
  "gene_symbol": "TASP1",
  "gene_name": "Threonine aspartase 1",
  "term_label": "cytoplasm",
  "gene": "UniProtKB:Q9H6P5"
}